{
  "term_label": "regulation of transcription by RNA polymerase II",
  "gene_symbol": "MED27",
  "gene": "UniProtKB:Q6P2C8",
  "gene_name": "Mediator of RNA polymerase II transcription subunit 27",
  "term_id": "GO:0006357"
}